{
  "gene_symbol": "AGXT",
  "gene_name": "Alanine--glyoxylate aminotransferase",
  "term_label": "peroxisome",
  "term_id": "GO:0005777",
  "gene": "UniProtKB:P21549"
}